{
  "gene_name": "Pumilio homolog 3",
  "gene": "UniProtKB:Q15397",
  "term_label": "mRNA binding",
  "term_id": "GO:0003729",
  "gene_symbol": "PUM3"
}